{
  "gene": "UniProtKB:Q9BVL2",
  "gene_symbol": "NUP58",
  "gene_name": "Nucleoporin p58_p45",
  "term_label": "nuclear localization sequence binding",
  "term_id": "GO:0008139"
}